histone deacetylase inhibitor activity [GO:0046811] (molecular function) References: PMID:10482575 Sources: GOC:ai Definition: Binds to and stops, prevents or reduces the activity of histone deacetylase, which catalyzes of the removal of acetyl groups from histones, proteins complexed to DNA in chromatin and chromosomes. Relationships: is a type of GO:0004857; is a type of histone deacetylase regulator activity [GO:0035033]; negatively regulates histone deacetylase activity [GO:0004407]